regulation of cholesterol transport [GO:0032374] (biological process) Subtypes: regulation of cholesterol efflux [GO:0010874], negative regulation of cholesterol transport [GO:0032375], positive regulation of cholesterol transport [GO:0032376], regulation of intracellular cholesterol transport [GO:0032383], GO:0060620, regulation of reverse cholesterol transport [GO:1903062] Sources: GOC:mah Relationships: is a type of GO:0032371; regulates cholesterol transport [GO:0030301] Definition: Any process that modulates the frequency, rate or extent of the directed movement of cholesterol into, out of or within a cell, or between cells, by means of some agent such as a transporter or pore.